{
  "term_label": "protein folding",
  "gene": "UniProtKB:P45877",
  "term_id": "GO:0006457",
  "gene_name": "Peptidyl-prolyl cis-trans isomerase C",
  "gene_symbol": "PPIC"
}